{
  "gene_name": "T cell receptor beta joining 2-2",
  "term_id": "UNKNOWN:0002",
  "gene_symbol": "TRBJ2-2",
  "gene": "UniProtKB:A0A0A0MT94",
  "term_label": "Unknown biological process"
}